{
  "gene_name": "Heat shock cognate 71 kDa protein",
  "gene_symbol": "HSPA8",
  "term_label": "cytoplasm",
  "term_id": "GO:0005737",
  "gene": "UniProtKB:P11142"
}